{
  "gene": "UniProtKB:A0A0B4J1U3",
  "gene_name": "Immunoglobulin lambda variable 1-36",
  "gene_symbol": "IGLV1-36",
  "term_label": "Unknown molecular function",
  "term_id": "UNKNOWN:0001"
}